phosphatidylinositol 3-kinase binding [GO:0043548] (molecular function) References: PMID:10209156, PMID:9255069 Subtypes: phosphatidylinositol 3-kinase regulatory subunit binding [GO:0036312], phosphatidylinositol 3-kinase catalytic subunit binding [GO:0036313] Definition: Binding to a phosphatidylinositol 3-kinase, any enzyme that catalyzes the addition of a phosphate group to an inositol lipid at the 3' position of the inositol ring. Relationships: is a type of protein binding [GO:0005515] Also known as: PI3K binding, phosphoinositide 3-kinase binding